{
  "term_label": "Unknown molecular function",
  "term_id": "UNKNOWN:0001",
  "gene_symbol": "CCDC160",
  "gene_name": "Coiled-coil domain-containing protein 160",
  "gene": "UniProtKB:A6NGH7"
}